{
  "term_label": "D-amino acid catabolic process",
  "term_id": "GO:0019478",
  "gene": "UniProtKB:Q99489",
  "gene_symbol": "DDO",
  "gene_name": "D-aspartate oxidase"
}